cytochrome-c peroxidase activity [GO:0004130] (molecular function) Definition: Catalysis of the reaction: 2 ferrocytochrome c + hydrogen peroxide = 2 ferricytochrome c + 2 H2O. Sources: EC:1.11.1.5 Relationships: is a type of GO:0004601 Also known as: apocytochrome c peroxidase activity, cytochrome c peroxidase activity, cytochrome c-551 peroxidase activity, cytochrome c-H2O oxidoreductase activity, cytochrome peroxidase activity, ferrocytochrome-c:hydrogen-peroxide oxidoreductase activity, mesocytochrome c peroxidase azide, mesocytochrome c peroxidase cyanate, mesocytochrome c peroxidase cyanide